{
  "gene_name": "Immunoglobulin kappa variable 1D-16",
  "gene_symbol": "IGKV1D-16",
  "term_label": "immunoglobulin complex",
  "gene": "UniProtKB:P01601",
  "term_id": "GO:0019814"
}